{
  "gene_name": "Putative uncharacterized protein encoded by LINC00588",
  "gene_symbol": "LINC00588",
  "term_id": "UNKNOWN:0003",
  "term_label": "Unknown cellular component",
  "gene": "UniProtKB:Q9Y4M8"
}